{
  "gene": "UniProtKB:O76024",
  "gene_symbol": "WFS1",
  "term_id": "UNKNOWN:0001",
  "term_label": "Unknown molecular function",
  "gene_name": "Wolframin"
}